{
  "term_id": "UNKNOWN:0001",
  "gene_name": "Putative uncharacterized protein FLJ42384",
  "gene": "UniProtKB:Q6ZVL8",
  "gene_symbol": "Q6ZVL8",
  "term_label": "Unknown molecular function"
}